{
  "gene": "UniProtKB:P02671",
  "gene_name": "Fibrinogen alpha chain",
  "gene_symbol": "FGA",
  "term_id": "GO:0042730",
  "term_label": "fibrinolysis"
}